{
  "term_label": "growth factor activity",
  "gene_name": "Ameloblastin",
  "term_id": "GO:0008083",
  "gene": "UniProtKB:Q9NP70",
  "gene_symbol": "AMBN"
}